distal tubule morphogenesis [GO:0072156] (biological process) Subtypes: pronephric distal tubule morphogenesis [GO:0039013], mesonephric distal tubule morphogenesis [GO:0061273], metanephric distal tubule morphogenesis [GO:0072287] Sources: GOC:mtg_kidney_jan10 Definition: The process in which the anatomical structures of a distal tubule are generated and organized. The distal tubule is a nephron tubule that begins at the macula densa and extends to the connecting tubule. Relationships: is a type of nephron tubule morphogenesis [GO:0072078]; is part of GO:0072017